{
  "gene": "UniProtKB:P25391",
  "gene_symbol": "LAMA1",
  "gene_name": "Laminin subunit alpha-1",
  "term_id": "GO:0007165",
  "term_label": "signal transduction"
}